{
  "term_id": "GO:0016020",
  "gene_name": "Potassium voltage-gated channel subfamily A member 3",
  "term_label": "membrane",
  "gene_symbol": "KCNA3",
  "gene": "UniProtKB:P22001"
}